pentraxin receptor activity [GO:0008029] (molecular function) Definition: Combining with a pentraxin and transmitting the signal from one side of the membrane to the other to initiate a change in cell activity. Subtypes: neuronal pentraxin receptor activity [GO:0008030] Sources: GOC:add, GOC:signaling, ISBN:0781735149 Note: Note that pentraxins include such proteins as serum amyloid P component (SAP) and C-reactive protein (CRP). Relationships: is a type of opsonin receptor activity [GO:0001847]; has part pentraxin binding [GO:0001864] Also known as: pentaxin receptor